{
  "gene_symbol": "TMTC4",
  "gene": "UniProtKB:Q5T4D3",
  "term_id": "GO:0030968",
  "term_label": "endoplasmic reticulum unfolded protein response",
  "gene_name": "Protein O-mannosyl-transferase TMTC4"
}